{
  "term_id": "GO:0005615",
  "gene": "UniProtKB:O95925",
  "term_label": "extracellular space",
  "gene_name": "Eppin",
  "gene_symbol": "EPPIN"
}